{
  "gene": "UniProtKB:A0A1W2PQ73",
  "gene_symbol": "ERFL",
  "gene_name": "ETS domain-containing transcription factor ERF-like",
  "term_id": "GO:0006357",
  "term_label": "regulation of transcription by RNA polymerase II"
}